{
  "term_id": "GO:0042742",
  "term_label": "defense response to bacterium",
  "gene_name": "Gasdermin-A",
  "gene_symbol": "GSDMA",
  "gene": "UniProtKB:Q96QA5"
}